{
  "term_label": "focal adhesion",
  "gene_name": "LIM and senescent cell antigen-like-containing domain protein 1",
  "gene_symbol": "LIMS1",
  "gene": "UniProtKB:P48059",
  "term_id": "GO:0005925"
}